{
  "gene_symbol": "PFKL",
  "term_id": "GO:0016020",
  "term_label": "membrane",
  "gene": "UniProtKB:P17858",
  "gene_name": "ATP-dependent 6-phosphofructokinase, liver type"
}